cleavage furrow ingression [GO:0036090] (biological process) Definition: Advancement of the cleavage furrow from the outside of the cell inward towards the center of the cell. The cleavage furrow acts as a 'purse string' which draws tight to separate daughter cells during cytokinesis and partition the cytoplasm between the two daughter cells. The furrow ingresses until a cytoplasmic bridge is formed. References: PMID:15811947, PMID:20687468 Also known as: cleavage furrow contraction Note: Consider also annotating to 'contractile ring contraction involved in cell cycle cytokinesis ; GO:0000916'. Relationships: is a type of GO:0032506; is a type of plasma membrane invagination [GO:0099024]; is part of cytoskeleton-dependent cytokinesis [GO:0061640] Subtypes: GO:1990386